{
  "gene_name": "Macrophage-stimulating protein receptor",
  "gene": "UniProtKB:Q04912",
  "gene_symbol": "MST1R",
  "term_label": "cell surface receptor protein tyrosine kinase signaling pathway",
  "term_id": "GO:0007169"
}